{
  "gene": "UniProtKB:P42830",
  "gene_name": "C-X-C motif chemokine 5",
  "gene_symbol": "CXCL5",
  "term_label": "antimicrobial humoral immune response mediated by antimicrobial peptide",
  "term_id": "GO:0061844"
}